fructosamine catabolic process [GO:0030392] (BP) Relationships: is a type of fructosamine metabolic process [GO:0030389]; is a type of amino sugar catabolic process [GO:0046348] Definition: The chemical reactions and pathways resulting in the breakdown of fructosamine, a fructose molecule containing an amino group in place of a hydroxyl group. Sources: GOC:jl, ISBN:0192801023 Also known as: fructosamine breakdown, fructosamine catabolism, fructosamine degradation Subtypes: fructoselysine catabolic process [GO:1901281]